{
  "term_label": "synaptic transmission, glutamatergic",
  "gene_symbol": "GRIA3",
  "term_id": "GO:0035249",
  "gene": "UniProtKB:P42263",
  "gene_name": "Glutamate receptor 3"
}